{
  "term_label": "neuron differentiation",
  "gene_symbol": "EMX1",
  "term_id": "GO:0030182",
  "gene_name": "Homeobox protein EMX1",
  "gene": "UniProtKB:Q04741"
}